{
  "gene_name": "Transcription factor HES-3",
  "term_id": "GO:0009952",
  "gene_symbol": "HES3",
  "gene": "UniProtKB:Q5TGS1",
  "term_label": "anterior/posterior pattern specification"
}